{
  "term_id": "UNKNOWN:0003",
  "gene": "UniProtKB:Q9UL59",
  "gene_name": "Zinc finger protein 214",
  "term_label": "Unknown cellular component",
  "gene_symbol": "ZNF214"
}